{
  "gene": "UniProtKB:Q13233",
  "gene_symbol": "MAP3K1",
  "term_label": "cytosol",
  "term_id": "GO:0005829",
  "gene_name": "Mitogen-activated protein kinase kinase kinase 1"
}